2-dehydro-3-deoxy-L-arabinonate dehydratase activity [GO:0047449] (molecular function) Definition: Catalysis of the reaction: 2-dehydro-3-deoxy-L-arabinonate = 2,5-dioxopentanoate + H2O. Relationships: is a type of GO:0016836 Also known as: 2-dehydro-3-deoxy-L-arabinonate hydro-lyase (2,5-dioxopentanoate-forming), 2-dehydro-3-deoxy-L-arabinonate hydro-lyase activity, 2-keto-3-deoxy-L-arabinonate dehydratase activity Sources: EC:4.2.1.43, RHEA:17201